oocyte fate commitment [GO:0048600] (biological process) Sources: GOC:go_curators Relationships: is a type of developmental process involved in reproduction [GO:0003006]; is a type of cell fate commitment [GO:0045165]; is part of oocyte differentiation [GO:0009994] Definition: The process in which the developmental fate of a cell becomes restricted such that it will develop into an oocyte.